{
  "gene_symbol": "SLC35B1",
  "gene_name": "Solute carrier family 35 member B1",
  "term_id": "GO:0072334",
  "gene": "UniProtKB:P78383",
  "term_label": "UDP-galactose transmembrane transport"
}